negative regulation of mitotic cell cycle phase transition [GO:1901991] (biological process) Subtypes: negative regulation of exit from mitosis [GO:0001100], negative regulation of G2/M transition of mitotic cell cycle [GO:0010972], mitotic cell size control checkpoint signaling [GO:0031567], negative regulation of mitotic metaphase/anaphase transition [GO:0045841], negative regulation of G1/S transition of mitotic cell cycle [GO:2000134] Also known as: down regulation of mitotic cell cycle phase transition, down-regulation of mitotic cell cycle phase transition, downregulation of mitotic cell cycle phase transition, inhibition of mitotic cell cycle phase transition Relationships: is a type of negative regulation of mitotic cell cycle [GO:0045930]; is a type of negative regulation of cell cycle phase transition [GO:1901988]; is a type of GO:1901990; negatively regulates mitotic cell cycle phase transition [GO:0044772] Definition: Any process that stops, prevents or reduces the frequency, rate or extent of mitotic cell cycle phase transition. References: PMID:22841721 Sources: GOC:TermGenie, GOC:mtg_cell_cycle